{
  "gene_symbol": "PLCD4",
  "gene_name": "1-phosphatidylinositol 4,5-bisphosphate phosphodiesterase delta-4",
  "term_label": "plasma membrane",
  "term_id": "GO:0005886",
  "gene": "UniProtKB:Q9BRC7"
}